acylcarnitine hydrolase activity [GO:0047619] (molecular function) Relationships: is a type of carboxylic ester hydrolase activity [GO:0052689] Also known as: HACH, O-acylcarnitine acylhydrolase activity, carnitine ester hydrolase activity, high activity acylcarnitine hydrolase activity, long-chain acyl-L-carnitine hydrolase activity, palmitoyl carnitine hydrolase activity, palmitoyl-L-carnitine hydrolase activity, palmitoylcarnitine hydrolase activity Sources: EC:3.1.1.28, MetaCyc:ACYLCARNITINE-HYDROLASE-RXN Definition: Catalysis of the reaction: O-acylcarnitine + H2O = a fatty acid + L-carnitine.